{
  "gene_name": "Structure-specific endonuclease subunit SLX4",
  "term_id": "GO:0000712",
  "gene_symbol": "SLX4",
  "term_label": "resolution of meiotic recombination intermediates",
  "gene": "UniProtKB:Q8IY92"
}